positive regulation of epithelial cell proliferation [GO:0050679] (biological process) Subtypes: positive regulation of endothelial cell proliferation [GO:0001938], positive regulation of keratinocyte proliferation [GO:0010838], positive regulation of mammary gland epithelial cell proliferation [GO:0033601], positive regulation of urothelial cell proliferation [GO:0050677], positive regulation of epithelial cell proliferation involved in wound healing [GO:0060054], positive regulation of epithelial cell proliferation involved in lung morphogenesis [GO:0060501], positive regulation of epithelial cell proliferation involved in prostate gland development [GO:0060769], positive regulation of synoviocyte proliferation [GO:1901647], positive regulation of sebum secreting cell proliferation [GO:1904004], positive regulation of cholangiocyte proliferation [GO:1904056], GO:1904197, GO:1904443, positive regulation of type B pancreatic cell proliferation [GO:1904692], positive regulation of acinar cell proliferation [GO:1904699], GO:2000347, positive regulation of lens epithelial cell proliferation [GO:2001111] Definition: Any process that activates or increases the rate or extent of epithelial cell proliferation. Also known as: up regulation of epithelial cell proliferation, up-regulation of epithelial cell proliferation, upregulation of epithelial cell proliferation, activation of epithelial cell proliferation, stimulation of epithelial cell proliferation Sources: GOC:ai Relationships: is a type of positive regulation of cell population proliferation [GO:0008284]; is a type of regulation of epithelial cell proliferation [GO:0050678]; positively regulates epithelial cell proliferation [GO:0050673]